{
  "term_label": "Unknown molecular function",
  "gene_name": "Cytochrome P450 4Z1",
  "gene": "UniProtKB:Q86W10",
  "term_id": "UNKNOWN:0001",
  "gene_symbol": "CYP4Z1"
}